{
  "gene": "UniProtKB:A6NNX1",
  "term_label": "Unknown cellular component",
  "term_id": "UNKNOWN:0003",
  "gene_symbol": "RIIAD1",
  "gene_name": "RIIa domain-containing protein 1"
}